{
  "term_label": "L-type voltage-gated calcium channel complex",
  "gene": "UniProtKB:Q9BXT2",
  "term_id": "GO:1990454",
  "gene_symbol": "CACNG6",
  "gene_name": "Voltage-dependent calcium channel gamma-6 subunit"
}